{
  "term_id": "GO:0005643",
  "gene": "UniProtKB:Q8TEM1",
  "term_label": "nuclear pore",
  "gene_name": "Nuclear pore membrane glycoprotein 210",
  "gene_symbol": "NUP210"
}